{
  "term_id": "GO:0006281",
  "gene_name": "Ubiquitin-conjugating enzyme E2 A",
  "gene": "UniProtKB:P49459",
  "gene_symbol": "UBE2A",
  "term_label": "DNA repair"
}